{
  "gene_name": "Kelch-like protein 2",
  "term_id": "GO:0031463",
  "gene": "UniProtKB:O95198",
  "term_label": "Cul3-RING ubiquitin ligase complex",
  "gene_symbol": "KLHL2"
}